{
  "term_label": "cytoplasm",
  "gene_symbol": "MYH4",
  "gene_name": "Myosin-4",
  "gene": "UniProtKB:Q9Y623",
  "term_id": "GO:0005737"
}